protein ufmylation [GO:0071569] (biological process) Relationships: is a type of protein modification by small protein conjugation [GO:0032446] References: PMID:20018847 Sources: GOC:vw Definition: Covalent attachment of the ubiquitin-like protein UFM1 to another protein. Subtypes: protein polyufmylation [GO:1990564]